{
  "term_id": "GO:0007015",
  "gene": "UniProtKB:Q92730",
  "term_label": "actin filament organization",
  "gene_symbol": "RND1",
  "gene_name": "Rho-related GTP-binding protein Rho6"
}